{
  "gene_name": "Protein odd-skipped-related 1",
  "gene": "UniProtKB:Q8TAX0",
  "term_id": "GO:0001655",
  "term_label": "urogenital system development",
  "gene_symbol": "OSR1"
}